benzoin aldolase activity [GO:0047695] (molecular function) Sources: EC:4.1.2.38, RHEA:21460 Also known as: 2-hydroxy-1,2-diphenylethanone benzaldehyde-lyase 2-hydroxy-1,2- activity, 2-hydroxy-1,2-diphenylethanone benzaldehyde-lyase 2-hydroxy-1,2-diphenylethanone benzaldehyde-lyase (benzaldehyde-forming), 2-hydroxy-1,2-diphenylethanone benzaldehyde-lyase 2-hydroxy-1,2-diphenylethanone benzaldehyde-lyase activity, benzaldehyde lyase activity, diphenylethanone benzaldehyde-lyase activity Relationships: is a type of aldehyde-lyase activity [GO:0016832] Definition: Catalysis of the reaction: benzoin = 2 benzaldehyde.